regulation of mRNA metabolic process [GO:1903311] (biological process) Relationships: is a type of regulation of RNA metabolic process [GO:0051252]; regulates mRNA metabolic process [GO:0016071] Subtypes: regulation of mRNA processing [GO:0050684], GO:0061013, regulation of mRNA modification [GO:0090365], GO:1901834, GO:1903312, positive regulation of mRNA metabolic process [GO:1903313] Definition: Any process that modulates the frequency, rate or extent of mRNA metabolic process. Also known as: regulation of mRNA metabolism Sources: GOC:TermGenie, GOC:vw, GO_REF:0000058